{
  "term_id": "GO:0016592",
  "term_label": "mediator complex",
  "gene": "UniProtKB:Q8TDQ0",
  "gene_name": "Hepatitis A virus cellular receptor 2",
  "gene_symbol": "HAVCR2"
}